regulation of ATPase-coupled calcium transmembrane transporter activity [GO:1901894] (biological process) Relationships: is a type of GO:0022898; is a type of regulation of ATP-dependent activity [GO:0043462]; regulates P-type calcium transporter activity [GO:0005388] Also known as: regulation of calcium pump, regulation of ATP phosphohydrolase (Ca2+-transporting), regulation of Ca(2+)-transporting ATPase activity, regulation of Ca2+-pumping ATPase activity, regulation of Ca2+-transporting ATPase activity, regulation of calcium transporting ATPase activity, regulation of calcium-transporting ATPase activity, regulation of calcium ABC transporter, regulation of calcium efflux ATPase, regulation of calcium-translocating P-type ATPase activity, regulation of plasma membrane Ca-ATPase, regulation of sarco(endo)plasmic reticulum Ca2+-ATPase, regulation of sarcoplasmic reticulum ATPase Definition: Any process that modulates the frequency, rate or extent of an ATPase-coupled calcium transmembrane transporter activity. References: PMID:19708671 Sources: GOC:BHF, GOC:TermGenie, GOC:rl Subtypes: negative regulation of ATPase-coupled calcium transmembrane transporter activity [GO:1901895], GO:1901896